{
  "gene_symbol": "KMT2E",
  "term_label": "Rpd3L-Expanded complex",
  "gene_name": "Inactive histone-lysine N-methyltransferase 2E",
  "gene": "UniProtKB:Q8IZD2",
  "term_id": "GO:0070210"
}